{
  "gene_name": "Zinc finger X-linked protein ZXDB",
  "term_id": "GO:0006357",
  "term_label": "regulation of transcription by RNA polymerase II",
  "gene_symbol": "ZXDB",
  "gene": "UniProtKB:P98169"
}